{
  "gene": "UniProtKB:P43681",
  "term_label": "plasma membrane",
  "gene_name": "Neuronal acetylcholine receptor subunit alpha-4",
  "term_id": "GO:0005886",
  "gene_symbol": "CHRNA4"
}